{
  "term_label": "detection of chemical stimulus involved in sensory perception of smell",
  "term_id": "GO:0050911",
  "gene_symbol": "OR2J2",
  "gene": "UniProtKB:O76002",
  "gene_name": "Olfactory receptor 2J2"
}